{
  "term_label": "regulation of cell shape",
  "term_id": "GO:0008360",
  "gene_symbol": "FMNL2",
  "gene": "UniProtKB:Q96PY5",
  "gene_name": "Formin-like protein 2"
}